{
  "term_label": "nuclear speck",
  "gene": "UniProtKB:P84103",
  "gene_name": "Serine_arginine-rich splicing factor 3",
  "term_id": "GO:0016607",
  "gene_symbol": "SRSF3"
}